{
  "term_label": "Unknown molecular function",
  "term_id": "UNKNOWN:0001",
  "gene": "UniProtKB:Q14517",
  "gene_name": "Protocadherin Fat 1",
  "gene_symbol": "FAT1"
}